{
  "term_label": "hydroxymethylglutaryl-CoA lyase activity",
  "gene": "UniProtKB:P35914",
  "gene_symbol": "HMGCL",
  "gene_name": "Hydroxymethylglutaryl-CoA lyase, mitochondrial",
  "term_id": "GO:0004419"
}